establishment or maintenance of polarity of embryonic epithelium [GO:0016332] (biological process) Subtypes: maintenance of polarity of embryonic epithelium [GO:0042250] Definition: Any cellular process that results in the specification, formation or maintenance of anisotropic intracellular organization of epithelial cells in an embryo. Sources: GOC:isa_complete, GOC:mah Relationships: is a type of establishment or maintenance of cell polarity [GO:0007163]; is part of morphogenesis of embryonic epithelium [GO:0016331]